anthocyanidin 3-O-glucoside 2''-O-glucosyltransferase activity [GO:0102455] (molecular function) Sources: GOC:pz, RHEA:35419 Definition: Catalysis of the reaction: UDP-alpha-D-glucose + an anthocyanidin-3-O-beta-D-glucoside = UDP + H+ + an anthocyanidin 3-O-sophoroside. Relationships: is a type of GO:0016758